{
  "gene_name": "Endophilin-A3",
  "term_label": "presynapse",
  "gene": "UniProtKB:Q99963",
  "gene_symbol": "SH3GL3",
  "term_id": "GO:0098793"
}